{
  "gene": "UniProtKB:Q13591",
  "gene_symbol": "SEMA5A",
  "term_label": "semaphorin-plexin signaling pathway",
  "term_id": "GO:0071526",
  "gene_name": "Semaphorin-5A"
}